{
  "gene_symbol": "OGN",
  "term_label": "Unknown molecular function",
  "term_id": "UNKNOWN:0001",
  "gene": "UniProtKB:P20774",
  "gene_name": "Mimecan"
}